{
  "gene_name": "Histone-arginine methyltransferase METTL23",
  "gene_symbol": "METTL23",
  "term_label": "nucleus",
  "term_id": "GO:0005634",
  "gene": "UniProtKB:Q86XA0"
}